{
  "gene": "UniProtKB:Q9UDY8",
  "gene_symbol": "MALT1",
  "gene_name": "Mucosa-associated lymphoid tissue lymphoma translocation protein 1",
  "term_id": "GO:0004175",
  "term_label": "endopeptidase activity"
}